dUTP diphosphatase activity [GO:0004170] (molecular function) Definition: Catalysis of the reaction: dUTP + H2O = dUMP + H+ + diphosphate. Also known as: dUTP pyrophosphatase activity, dUTP nucleotidohydrolase activity, dUTPase activity, deoxyuridine-triphosphatase activity, desoxyuridine 5'-triphosphatase activity, desoxyuridine 5'-triphosphate nucleotidohydrolase activity Relationships: is a type of GO:0047429 Sources: RHEA:10248 Regulation: negatively regulated by dUTP pyrophosphatase inhibitor activity [GO:0004858]